{
  "gene_symbol": "CDH15",
  "gene_name": "Cadherin-15",
  "gene": "UniProtKB:P55291",
  "term_label": "adherens junction organization",
  "term_id": "GO:0034332"
}